positive regulation of autophagy of mitochondrion [GO:1903599] (biological process) Note: An example of this AMBRA1 - human (Q9C0C7) in PMID:21753002 inferred from direct assay Definition: Any process that activates or increases the frequency, rate or extent of mitochondrion degradation by autophagy. Relationships: is a type of GO:0010508; is a type of GO:1903146; positively regulates autophagy of mitochondrion [GO:0000422] References: PMID:21753002 Sources: GOC:PARL, GOC:TermGenie, GOC:autophagy, GOC:pad, GO_REF:0000058 Subtypes: GO:1901526 Also known as: positive regulation of mitochondrial degradation, up regulation of mitochondrion degradation, up-regulation of mitochondrion degradation, upregulation of mitochondrion degradation, up regulation of mitophagy, up-regulation of mitophagy, upregulation of mitophagy, activation of mitophagy, activation of mitochondrion degradation